epithelial cell fate determination, open tracheal system [GO:0007425] (BP) Also known as: tracheal cell fate determination, tracheal epithelial cell fate determination, tracheal placode cell fate determination References: PMID:11063940 Sources: GOC:mtg_sensu Definition: The cell fate determination process in which a cell becomes capable of differentiating autonomously into an epithelial cell within an open tracheal system regardless of its environment; upon determination, the cell fate cannot be reversed. Tracheal cells are set aside as 10 clusters of approximately 80 cells on each side of the embryo (termed tracheal placodes). An example of this is found in Drosophila melanogaster. Relationships: is a type of cell fate determination [GO:0001709]; is part of open tracheal system development [GO:0007424]